{
  "term_id": "UNKNOWN:0001",
  "gene_name": "Probable ATP-dependent RNA helicase DDX31",
  "gene_symbol": "DDX31",
  "term_label": "Unknown molecular function",
  "gene": "UniProtKB:Q9H8H2"
}